{
  "term_label": "protein serine/threonine kinase activity",
  "term_id": "GO:0004674",
  "gene_symbol": "WNK2",
  "gene": "UniProtKB:Q9Y3S1",
  "gene_name": "Serine_threonine-protein kinase WNK2"
}